3,4-dihydroxy-2-butanone-4-phosphate synthase activity [GO:0008686] (molecular function) Definition: Catalysis of the reaction: D-ribulose 5-phosphate = (2S)-2-hydroxy-3-oxobutyl phosphate + formate + H+. Sources: EC:4.1.99.12, RHEA:18457 Relationships: is a type of carbon-carbon lyase activity [GO:0016830]